{
  "gene": "UniProtKB:P46098",
  "gene_symbol": "HTR3A",
  "term_id": "GO:0007268",
  "term_label": "chemical synaptic transmission",
  "gene_name": "5-hydroxytryptamine receptor 3A"
}